sperm ejaculation [GO:0042713] (biological process) References: PMID:26385403 Sources: GOC:jl Definition: The expulsion of seminal fluid, thick white fluid containing spermatozoa, from the male genital tract. Relationships: is a type of multicellular organismal reproductive process [GO:0048609]; is part of insemination [GO:0007320]